{
  "gene_symbol": "DNAJC14",
  "gene": "UniProtKB:Q6Y2X3",
  "term_id": "GO:0050780",
  "term_label": "dopamine receptor binding",
  "gene_name": "DnaJ homolog subfamily C member 14"
}